root cap mucilage biosynthetic process [GO:0048355] (biological process) Relationships: is a type of mucilage biosynthetic process [GO:0010192] Sources: GOC:jid Definition: The chemical reactions and pathways resulting in the formation of mucilage that occur in the root cap; mucilage is normally synthesized during root growth. Also known as: root cap mucilage anabolism, root cap mucilage biosynthesis, root cap mucilage formation, root cap mucilage synthesis